{
  "gene": "UniProtKB:Q495Y8",
  "gene_symbol": "SPDYE2",
  "gene_name": "Speedy protein E2",
  "term_id": "GO:0019901",
  "term_label": "protein kinase binding"
}